{
  "gene_name": "Tyrosine aminotransferase",
  "term_id": "UNKNOWN:0003",
  "gene_symbol": "TAT",
  "term_label": "Unknown cellular component",
  "gene": "UniProtKB:P17735"
}